{
  "gene_name": "Refilin-B",
  "gene_symbol": "RFLNB",
  "gene": "UniProtKB:Q8N5W9",
  "term_id": "GO:0031005",
  "term_label": "filamin binding"
}